positive regulation of lamellocyte differentiation [GO:0035205] (biological process) Relationships: is_a GO:0035203; is_a positive regulation of hemocyte differentiation [GO:0045612]; positively regulates lamellocyte differentiation [GO:0035171] References: PMID:14734104 Definition: Any process that activates or increases the frequency, rate or extent of lamellocyte differentiation. Lamellocytes differentiate massively in the lymph glands after parasitization and are large flat cells devoted to encapsulation of invaders too large to be phagocytosed by plasmatocytes. Also known as: up regulation of lamellocyte differentiation, up-regulation of lamellocyte differentiation, upregulation of lamellocyte differentiation, activation of lamellocyte differentiation, stimulation of lamellocyte differentiation